{
  "gene_name": "Synaptotagmin-11",
  "term_label": "axon",
  "gene": "UniProtKB:Q9BT88",
  "gene_symbol": "SYT11",
  "term_id": "GO:0030424"
}